{
  "gene_name": "Transmembrane gamma-carboxyglutamic acid protein 1",
  "term_label": "serine-type endopeptidase activity",
  "term_id": "GO:0004252",
  "gene": "UniProtKB:O14668",
  "gene_symbol": "PRRG1"
}